{
  "term_label": "spindle microtubule",
  "gene_name": "Regulator of microtubule dynamics protein 1",
  "gene": "UniProtKB:Q96DB5",
  "gene_symbol": "RMDN1",
  "term_id": "GO:0005876"
}